primary sex determination [GO:0007538] (biological process) Sources: GOC:mah Definition: The sex determination process that results in the initial specification of sexual status of an individual organism. Relationships: is a type of GO:0007530; is part of GO:0007275 Subtypes: primary sex determination, soma [GO:0007539], primary sex determination, germ-line [GO:0007542]